{
  "gene_symbol": "LEUTX",
  "gene": "UniProtKB:A8MZ59",
  "term_label": "nucleus",
  "term_id": "GO:0005634",
  "gene_name": "Paired-like homeodomain transcription factor LEUTX"
}